endothelial cell development [GO:0001885] (biological process) Sources: GOC:dph Regulation: regulated by GO:1901550; negatively regulated by negative regulation of endothelial cell development [GO:1901551]; positively regulated by GO:1901552 Definition: The progression of an endothelial cell over time, from its formation to the mature structure. Relationships: is_a epithelial cell development [GO:0002064]; is part of endothelial cell differentiation [GO:0045446] Subtypes: establishment of blood-nerve barrier [GO:0008065], endocardial cell development [GO:0060958], establishment of endothelial barrier [GO:0061028]